{
  "gene_symbol": "GSE1",
  "term_label": "Unknown biological process",
  "term_id": "UNKNOWN:0002",
  "gene": "UniProtKB:Q14687",
  "gene_name": "Genetic suppressor element 1"
}